{
  "gene_name": "Dual specificity mitogen-activated protein kinase kinase 7",
  "term_id": "GO:0008545",
  "gene": "UniProtKB:O14733",
  "gene_symbol": "MAP2K7",
  "term_label": "JUN kinase kinase activity"
}